beta-glucoside transport [GO:0015759] (biological process) Definition: The directed movement of beta-glucosides into, out of or within a cell, or between cells, by means of some agent such as a transporter or pore. Beta-glucosides are glycosides in which the sugar group is a glucose residue, and the anomeric carbon of the bond is in a beta configuration. References: PMID:3034860, PMID:6756954 Sources: GOC:jl, ISBN:0198506732 Relationships: is a type of glucoside transport [GO:0042946] Subtypes: salicin transport [GO:0042948], arbutin transport [GO:0042949]